regulation of detection of glucose [GO:2000970] (biological process) Sources: GOC:BHF Subtypes: negative regulation of detection of glucose [GO:2000971], GO:2000972 Also known as: regulation of glucose detection, regulation of glucose perception, regulation of glucose sensing Relationships: is a type of regulation of response to stimulus [GO:0048583]; regulates detection of glucose [GO:0051594] Definition: Any process that modulates the frequency, rate or extent of detection of glucose.